{
  "term_label": "phosphatidylinositol-3-phosphate biosynthetic process",
  "term_id": "GO:0036092",
  "gene_name": "Phosphatidylinositol 4-phosphate 3-kinase C2 domain-containing subunit alpha",
  "gene": "UniProtKB:O00443",
  "gene_symbol": "PIK3C2A"
}